{
  "term_label": "acetylcholine-gated channel complex",
  "gene_name": "Neuronal acetylcholine receptor subunit alpha-4",
  "gene": "UniProtKB:P43681",
  "term_id": "GO:0005892",
  "gene_symbol": "CHRNA4"
}